{
  "term_label": "Unknown biological process",
  "gene_name": "DnaJ homolog subfamily C member 4",
  "gene": "UniProtKB:Q9NNZ3",
  "gene_symbol": "DNAJC4",
  "term_id": "UNKNOWN:0002"
}